{
  "gene_symbol": "HSP90AA2P",
  "term_label": "cellular response to heat",
  "gene": "UniProtKB:Q14568",
  "term_id": "GO:0034605",
  "gene_name": "Heat shock protein HSP 90-alpha A2"
}